olfactory nerve morphogenesis [GO:0021627] (biological process) Sources: GOC:cls, GOC:dgh, GOC:dph, GOC:jid, GO_REF:0000021 Definition: The process in which the anatomical structure of the olfactory nerve is generated and organized. The olfactory nerve is a collection of sensory nerve rootlets that extend down from the olfactory bulb to the olfactory mucosa of the upper parts of the nasal cavity. This nerve conducts odor information to the brainstem. Also known as: CN I morphogenesis Relationships: is a type of cranial nerve morphogenesis [GO:0021602]; is part of olfactory nerve development [GO:0021553]